{
  "term_label": "anterograde synaptic vesicle transport",
  "gene": "UniProtKB:O14617",
  "gene_name": "AP-3 complex subunit delta-1",
  "gene_symbol": "AP3D1",
  "term_id": "GO:0048490"
}